negative regulation of mesodermal cell differentiation [GO:1905771] (biological process) References: PMID:23765923 Sources: GOC:BHF, GOC:BHF_miRNA, GOC:TermGenie, GOC:rph, GO_REF:0000058 Subtypes: GO:0042662 Definition: Any process that stops, prevents or reduces the frequency, rate or extent of mesodermal cell differentiation. Also known as: down regulation of mesoderm cell differentiation, down regulation of mesodermal cell differentiation, down-regulation of mesoderm cell differentiation, down-regulation of mesodermal cell differentiation, downregulation of mesoderm cell differentiation, downregulation of mesodermal cell differentiation, negative regulation of mesoderm cell differentiation, inhibition of mesoderm cell differentiation, inhibition of mesodermal cell differentiation Relationships: is a type of negative regulation of cell differentiation [GO:0045596]; is a type of regulation of mesodermal cell differentiation [GO:1905770]; negatively regulates mesodermal cell differentiation [GO:0048333]